{
  "term_label": "Golgi membrane",
  "gene": "UniProtKB:A6NH52",
  "gene_symbol": "TVP23A",
  "term_id": "GO:0000139",
  "gene_name": "Golgi apparatus membrane protein TVP23 homolog A"
}